RNA polymerase II CTD heptapeptide repeat peptidyl-prolyl isomerase activity [GO:0140838] (molecular function) Subtypes: RNA polymerase II CTD heptapeptide repeat P3 isomerase activity [GO:0140839], RNA polymerase II CTD heptapeptide repeat P6 isomerase activity [GO:0140840] References: PMID:28248323 Relationships: is a type of GO:0003755; is a type of RNA polymerase II CTD heptapeptide repeat modifying activity [GO:0140994] Definition: Catalysis of the reaction: RNA polymerase II large subunit CTD heptapeptide repeat (consensus YSPTSPS) cis-proline (omega=180) = RNA polymerase II large subunit trans-proline (omega=0).